{
  "gene_symbol": "PLPP5",
  "gene": "UniProtKB:Q8NEB5",
  "term_label": "phosphatidate phosphatase activity",
  "term_id": "GO:0008195",
  "gene_name": "Phospholipid phosphatase 5"
}